{
  "gene_name": "Acetylcholine receptor subunit alpha",
  "gene_symbol": "CHRNA1",
  "gene": "UniProtKB:P02708",
  "term_label": "skeletal muscle contraction",
  "term_id": "GO:0003009"
}